{
  "term_id": "GO:0000146",
  "gene_name": "Myosin-3",
  "gene": "UniProtKB:P11055",
  "gene_symbol": "MYH3",
  "term_label": "microfilament motor activity"
}